{
  "term_id": "GO:0043162",
  "term_label": "ubiquitin-dependent protein catabolic process via the multivesicular body sorting pathway",
  "gene_name": "Vacuolar protein sorting-associated protein 37A",
  "gene_symbol": "VPS37A",
  "gene": "UniProtKB:Q8NEZ2"
}